Kibra-Ex-Mer complex [GO:0036375] (cellular component) Also known as: KEM complex, Kbr, Ex and Mer complex Relationships: is a type of protein-containing complex [GO:0032991]; is part of apical part of cell [GO:0045177] Definition: An apical protein complex that contains the proteins Kibra, Expanded and Merlin (Mer), or orthologs thereof. In humans, the complex contains KIBRA, FDM6 and NF2. References: PMID:20159598